telencephalon astrocyte cell migration [GO:0022031] (biological process) Definition: The orderly movement of an astrocyte cell through the telencephalon. Sources: GOC:cls, GOC:dgh, GOC:dph, GOC:jid, GO_REF:0000021 Relationships: is a type of telencephalon glial cell migration [GO:0022030]; is a type of astrocyte cell migration [GO:0043615]